{
  "gene_name": "Ferroptosis suppressor protein 1",
  "gene": "UniProtKB:Q9BRQ8",
  "term_label": "mitochondrial membrane",
  "term_id": "GO:0031966",
  "gene_symbol": "AIFM2"
}